{
  "gene": "UniProtKB:Q9NZ71",
  "gene_name": "Regulator of telomere elongation helicase 1",
  "term_label": "DNA polymerase binding",
  "gene_symbol": "RTEL1",
  "term_id": "GO:0070182"
}